{
  "term_id": "GO:0038109",
  "gene_name": "Mast_stem cell growth factor receptor Kit",
  "gene": "UniProtKB:P10721",
  "gene_symbol": "KIT",
  "term_label": "Kit signaling pathway"
}